{
  "term_label": "mitochondrial inner membrane",
  "term_id": "GO:0005743",
  "gene_name": "Mitochondrial import inner membrane translocase subunit Tim10 B",
  "gene_symbol": "TIMM10B",
  "gene": "UniProtKB:Q9Y5J6"
}